{
  "gene": "UniProtKB:O43854",
  "term_id": "UNKNOWN:0001",
  "term_label": "Unknown molecular function",
  "gene_name": "EGF-like repeat and discoidin I-like domain-containing protein 3",
  "gene_symbol": "EDIL3"
}